phosphatidylserine lysophospholipase activity [GO:0120560] (molecular function) Relationships: is a type of GO:0120558 Also known as: phosphatidylserine sn-1 acylhydrolase, phosphatidylserine-specific phospholipase A1 Definition: Catalysis of the reaction: a 1-acyl-sn-glycero-3-phospho-L-serine + H2O = sn-glycero-3-phospho-L-serine + a fatty acid + H+. Sources: RHEA:32979